{
  "gene_symbol": "TMEM97",
  "term_id": "UNKNOWN:0001",
  "gene_name": "Sigma intracellular receptor 2",
  "term_label": "Unknown molecular function",
  "gene": "UniProtKB:Q5BJF2"
}